detection of chemical stimulus involved in sensory perception of sour taste [GO:0001581] (biological process) Definition: The series of events required for a sour taste stimulus to be received and converted to a molecular signal. Also known as: perception of sour taste, detection of chemical stimulus, perception of sour taste, sensory transduction of chemical stimulus, sensory detection of chemical stimulus during perception of sour taste, sensory detection of sour taste, sensory transduction of chemical stimulus during perception of sour taste, sensory transduction of sour taste, sour taste detection Relationships: is a type of detection of chemical stimulus involved in sensory perception of taste [GO:0050912]; is part of sensory perception of sour taste [GO:0050915] Sources: GOC:go_curators